cellular response to gonadotropin-releasing hormone [GO:0097211] (biological process) Definition: Any process that results in a change in state or activity of a cell (in terms of movement, secretion, enzyme production, gene expression, etc.) as a result of a gonadotropin-releasing hormone stimulus. Gonadotropin-releasing hormone (GnRH) is a peptide hormone responsible for the release of follicle-stimulating hormone (FSH) and luteinizing hormone (LH) from the anterior pituitary. GnRH is synthesized and released by the hypothalamus. Also known as: cellular response to GnRH, cellular response to gonadotrophin-releasing hormone Relationships: is a type of cellular response to peptide hormone stimulus [GO:0071375]; is a type of response to gonadotropin-releasing hormone [GO:0097210] References: PMID:15976007 Sources: GOC:yaf